{
  "gene": "UniProtKB:Q6PH81",
  "gene_symbol": "C16orf87",
  "term_id": "UNKNOWN:0001",
  "gene_name": "UPF0547 protein C16orf87",
  "term_label": "Unknown molecular function"
}